{
  "term_id": "GO:0000123",
  "gene_name": "Protein Jade-3",
  "gene": "UniProtKB:Q92613",
  "term_label": "histone acetyltransferase complex",
  "gene_symbol": "JADE3"
}